adenine/cytosine mispair binding [GO:0032136] (molecular function) Also known as: A/C mispair binding, C/A mispair binding, cytosine/adenine mispair binding Sources: GOC:vk Definition: Binding to a double-stranded DNA region containing an A/C mispair. Relationships: is a type of GO:0030983